phenylpropanoid catabolic process [GO:0046271] (biological process) Relationships: is a type of GO:0009056; is a type of phenylpropanoid metabolic process [GO:0009698] Also known as: phenylpropanoid breakdown, phenylpropanoid catabolism, phenylpropanoid degradation Subtypes: eugenol catabolic process [GO:0042856], coumarin catabolic process [GO:0046226], lignan catabolic process [GO:0046273], lignin catabolic process [GO:0046274], chalcone catabolic process [GO:0046280], cinnamic acid catabolic process [GO:0046281], GO:0046282, GO:0046288 Sources: GOC:ai Definition: The chemical reactions and pathways resulting in the breakdown of aromatic derivatives of trans-cinnamic acid.